regulation of mitochondrial membrane permeability [GO:0046902] (biological process) Subtypes: positive regulation of mitochondrial membrane permeability [GO:0035794], negative regulation of mitochondrial membrane permeability [GO:0035795], regulation of mitochondrial outer membrane permeabilization involved in apoptotic signaling pathway [GO:1901028], GO:1902108, GO:1902445 Sources: GOC:bf Also known as: regulation of transport across mitochondrial membrane, regulation of mitochondrial envelope permeability Relationships: is a type of GO:0007006; is a type of regulation of membrane permeability [GO:0090559]; is part of GO:0006839 Definition: Any process that modulates the frequency, rate or extent of the passage or uptake of molecules by the mitochondrial membrane.